{
  "gene": "UniProtKB:O14733",
  "gene_symbol": "MAP2K7",
  "gene_name": "Dual specificity mitogen-activated protein kinase kinase 7",
  "term_id": "UNKNOWN:0003",
  "term_label": "Unknown cellular component"
}